plasmacytoid dendritic cell differentiation involved in immune response [GO:0002272] (BP) Definition: The process in which an immature plasmacytoid dendritic cell acquires the specialized features of a mature plasmacytoid dendritic cell contributing to an immune response. References: PMID:15990333 Sources: GOC:add Also known as: plasmacytoid dendritic cell differentiation during immune response Relationships: is a type of plasmacytoid dendritic cell activation involved in immune response [GO:0002271]; is a type of plasmacytoid dendritic cell differentiation [GO:0002273]